glycine:proton antiporter activity [GO:0140799] (molecular function) Relationships: is a type of GO:0015078; is a type of glycine transmembrane transporter activity [GO:0015187]; is a type of amino acid:monoatomic cation antiporter activity [GO:0140848] References: PMID:16701208, PMID:26912364 Definition: Enables the transfer of a solute or solutes from one side of a membrane to the other according to the reaction: glycine(out) + H+(in) = glycine(in) + H+(out).